dehydrogluconokinase activity [GO:0047841] (molecular function) Also known as: dehydogluconokinase activity, 2-ketogluconate kinase activity, 2-ketogluconokinase activity, ATP:2-dehydro-D-gluconate 6-phosphotransferase activity, ketogluconokinase (phosphorylating), ketogluconokinase activity Definition: Catalysis of the reaction: 2-dehydro-D-gluconate + ATP = 6-phospho-2-dehydro-D-gluconate + ADP + 2 H+. Sources: EC:2.7.1.13, RHEA:10788 Relationships: is_a kinase activity [GO:0016301]; is a type of phosphotransferase activity, alcohol group as acceptor [GO:0016773]